{
  "gene_name": "Chloride channel protein ClC-Kb",
  "gene": "UniProtKB:P51801",
  "term_id": "GO:0005886",
  "term_label": "plasma membrane",
  "gene_symbol": "CLCNKB"
}